{
  "gene": "UniProtKB:O95747",
  "gene_symbol": "OXSR1",
  "gene_name": "Serine_threonine-protein kinase OSR1",
  "term_id": "GO:0071474",
  "term_label": "cellular hyperosmotic response"
}